{
  "term_label": "Unknown cellular component",
  "gene_symbol": "KRTAP16-1",
  "gene_name": "Keratin-associated protein 16-1",
  "gene": "UniProtKB:A8MUX0",
  "term_id": "UNKNOWN:0003"
}